{
  "gene_symbol": "SLC2A10",
  "gene": "UniProtKB:O95528",
  "term_label": "circulatory system development",
  "term_id": "GO:0072359",
  "gene_name": "Solute carrier family 2, facilitated glucose transporter member 10"
}